{
  "term_id": "GO:0071230",
  "gene": "UniProtKB:Q6IAA8",
  "gene_name": "Ragulator complex protein LAMTOR1",
  "gene_symbol": "LAMTOR1",
  "term_label": "cellular response to amino acid stimulus"
}